{
  "term_id": "GO:0009897",
  "gene_symbol": "RTBDN",
  "term_label": "external side of plasma membrane",
  "gene_name": "Retbindin",
  "gene": "UniProtKB:Q9BSG5"
}